{
  "gene_name": "NEDD8-conjugating enzyme Ubc12",
  "gene": "UniProtKB:P61081",
  "term_label": "protein neddylation",
  "gene_symbol": "UBE2M",
  "term_id": "GO:0045116"
}